positive regulation of cell migration involved in sprouting angiogenesis [GO:0090050] (biological process) Sources: GOC:BHF, GOC:dph, GOC:rl, GOC:tb Relationships: is a type of positive regulation of blood vessel endothelial cell migration [GO:0043536]; is a type of regulation of cell migration involved in sprouting angiogenesis [GO:0090049]; positively regulates cell migration involved in sprouting angiogenesis [GO:0002042] Definition: Any process that increases the frequency, rate or extent of cell migration involved in sprouting angiogenesis. Cell migration involved in sprouting angiogenesis is the orderly movement of endothelial cells into the extracellular matrix in order to form new blood vessels contributing to the process of sprouting angiogenesis.